regulation of lamellipodium assembly [GO:0010591] (biological process) Definition: Any process that modulates the rate, frequency or extent of the formation of a lamellipodium, a thin sheetlike extension of the surface of a migrating cell. Sources: GOC:dph, GOC:tb Also known as: regulation of lamellipodium biogenesis Relationships: is a type of GO:0120032; is a type of GO:1902743; regulates lamellipodium assembly [GO:0030032] Subtypes: positive regulation of lamellipodium assembly [GO:0010592], negative regulation of lamellipodium assembly [GO:0010593]